negative regulation of B cell apoptotic process [GO:0002903] (biological process) Definition: Any process that stops, prevents, or reduces the frequency, rate, or extent of B cell apoptotic process. Sources: GOC:add, GOC:mtg_apoptosis Also known as: down regulation of B cell apoptosis, down-regulation of B cell apoptosis, downregulation of B cell apoptosis, inhibition of B cell apoptosis, negative regulation of B cell apoptosis Relationships: is a type of regulation of B cell apoptotic process [GO:0002902]; is a type of negative regulation of lymphocyte apoptotic process [GO:0070229]; negatively regulates B cell apoptotic process [GO:0001783] Subtypes: GO:0002868, negative regulation of mature B cell apoptotic process [GO:0002906]